response to glycoprotein [GO:1904587] (biological process) Definition: Any process that results in a change in state or activity of a cell or an organism (in terms of movement, secretion, enzyme production, gene expression, etc.) as a result of a glycoprotein stimulus. Relationships: is a type of response to nitrogen compound [GO:1901698]; is a type of response to oxygen-containing compound [GO:1901700] Subtypes: ubiquitin-dependent glycoprotein ERAD pathway [GO:0097466], GO:1904400, cellular response to glycoprotein [GO:1904588] References: PMID:14597422 Sources: GOC:TermGenie, GO_REF:0000071 Also known as: response to glycoproteins